{
  "gene_name": "CCAAT_enhancer-binding protein delta",
  "term_id": "GO:0045595",
  "term_label": "regulation of cell differentiation",
  "gene_symbol": "CEBPD",
  "gene": "UniProtKB:P49716"
}